{
  "gene_symbol": "USP8",
  "gene": "UniProtKB:P40818",
  "term_label": "postsynaptic density",
  "gene_name": "Ubiquitin carboxyl-terminal hydrolase 8",
  "term_id": "GO:0014069"
}